{
  "term_label": "ciliary membrane",
  "term_id": "GO:0060170",
  "gene_symbol": "TMEM231",
  "gene": "UniProtKB:Q9H6L2",
  "gene_name": "Transmembrane protein 231"
}